response to cholesterol [GO:0070723] (biological process) Sources: GOC:BHF, GOC:vk Relationships: is a type of response to sterol [GO:0036314]; is a type of response to alcohol [GO:0097305] Subtypes: cellular response to cholesterol [GO:0071397] Definition: Any process that results in a change in state or activity of a cell or an organism (in terms of movement, secretion, enzyme production, gene expression, etc.) as a result of a cholesterol stimulus.